cyclin D2-CDK6 complex [GO:0097132] (cellular component) References: PMID:15935619 Sources: GOC:so Definition: A protein complex consisting of cyclin D2 and cyclin-dependent kinase 6 (CDK6). Cyclins are characterized by periodicity in protein abundance throughout the cell cycle. Cyclin-dependent kinases represent a family of serine/threonine protein kinases that become active upon binding to a cyclin regulatory partner. Relationships: is a type of GO:0000307